{
  "gene_name": "Glutamine-dependent NAD(+) synthetase",
  "term_id": "GO:0005737",
  "term_label": "cytoplasm",
  "gene_symbol": "NADSYN1",
  "gene": "UniProtKB:Q6IA69"
}